{
  "term_label": "Unknown molecular function",
  "gene_name": "Solute carrier family 35 member G6",
  "gene": "UniProtKB:P0C7Q6",
  "gene_symbol": "SLC35G6",
  "term_id": "UNKNOWN:0001"
}